{
  "gene_name": "Peptidyl-prolyl cis-trans isomerase FKBP14",
  "gene": "UniProtKB:Q9NWM8",
  "term_id": "UNKNOWN:0003",
  "term_label": "Unknown cellular component",
  "gene_symbol": "FKBP14"
}